{
  "term_label": "potassium ion transmembrane transport",
  "gene_symbol": "KCNH8",
  "gene_name": "Potassium voltage-gated channel subfamily H member 8",
  "term_id": "GO:0071805",
  "gene": "UniProtKB:Q96L42"
}